{
  "gene_symbol": "EML6",
  "term_id": "UNKNOWN:0003",
  "gene_name": "Echinoderm microtubule-associated protein-like 6",
  "term_label": "Unknown cellular component",
  "gene": "UniProtKB:Q6ZMW3"
}